{
  "gene_symbol": "CD79B",
  "term_id": "GO:0019815",
  "gene_name": "B-cell antigen receptor complex-associated protein beta chain",
  "term_label": "B cell receptor complex",
  "gene": "UniProtKB:P40259"
}